{
  "gene_name": "Sorting nexin-1",
  "gene": "UniProtKB:Q13596",
  "term_label": "early endosome to Golgi transport",
  "gene_symbol": "SNX1",
  "term_id": "GO:0034498"
}